fatty acid elongation [GO:0030497] (biological process) Subtypes: fatty acid elongation, saturated fatty acid [GO:0019367], fatty acid elongation, unsaturated fatty acid [GO:0019368] Relationships: is a type of fatty acid biosynthetic process [GO:0006633] Sources: ISBN:0716720094 Definition: The elongation of a fatty acid chain by the sequential addition of two-carbon units.